{
  "term_label": "triacyl lipopeptide binding",
  "gene": "UniProtKB:O60603",
  "gene_symbol": "TLR2",
  "term_id": "GO:0042497",
  "gene_name": "Toll-like receptor 2"
}